IgD immunoglobulin complex [GO:0071738] (CC) Relationships: is_a GO:0019814 Subtypes: IgD immunoglobulin complex, circulating [GO:0071739], IgD B cell receptor complex [GO:0071740], IgD immunoglobulin complex, GPI-anchored [GO:0071741] References: PMID:11282392 Sources: GOC:add, ISBN:0781765196 Note: Note that an IgD immunoglobulin complex has the function of antigen binding if a suitable antigen is available. Definition: A protein complex composed of two identical immunoglobulin heavy chains of the IgD isotype and two identical immunoglobulin light chains, held together by disulfide bonds. An IgD immunoglobulin complex may be embedded in the plasma membrane or present in the extracellular space, in mucosal areas or other tissues, or circulating in the blood or lymph.